{
  "term_id": "GO:1990116",
  "gene_symbol": "NEMF",
  "term_label": "ribosome-associated ubiquitin-dependent protein catabolic process",
  "gene": "UniProtKB:O60524",
  "gene_name": "Ribosome quality control complex subunit NEMF"
}